{
  "gene_symbol": "KIF18A",
  "gene": "UniProtKB:Q8NI77",
  "term_id": "GO:0007018",
  "term_label": "microtubule-based movement",
  "gene_name": "Kinesin-like protein KIF18A"
}